mesenchymal cell development [GO:0014031] (BP) Definition: The process aimed at the progression of a mesenchymal cell over time, from initial commitment of the cell to its specific fate, to the fully functional differentiated cell. Relationships: is a type of cell development [GO:0048468]; is part of mesenchymal cell differentiation [GO:0048762] Sources: GOC:dh, GOC:ef